{
  "gene_name": "Probable small intestine urate exporter",
  "gene": "UniProtKB:Q9Y2C5",
  "term_id": "GO:0044341",
  "gene_symbol": "SLC17A4",
  "term_label": "sodium-dependent phosphate transport"
}